{
  "term_label": "Unknown biological process",
  "gene": "UniProtKB:Q86TP1",
  "term_id": "UNKNOWN:0002",
  "gene_name": "Exopolyphosphatase PRUNE1",
  "gene_symbol": "PRUNE1"
}